positive regulation of chanoclavine-I aldehyde biosynthetic process [GO:1900648] (biological process) Definition: Any process that activates or increases the frequency, rate or extent of chanoclavine-I aldehyde biosynthetic process. Sources: GOC:TermGenie, GOC:di Also known as: activation of chanoclavine-I aldehyde anabolism, activation of chanoclavine-I aldehyde biosynthesis, activation of chanoclavine-I aldehyde formation, activation of chanoclavine-I aldehyde synthesis, positive regulation of chanoclavine-I aldehyde anabolism, positive regulation of chanoclavine-I aldehyde biosynthesis, positive regulation of chanoclavine-I aldehyde formation, positive regulation of chanoclavine-I aldehyde synthesis, up regulation of chanoclavine-I aldehyde anabolism, up regulation of chanoclavine-I aldehyde biosynthesis, up regulation of chanoclavine-I aldehyde biosynthetic process, up regulation of chanoclavine-I aldehyde formation, up regulation of chanoclavine-I aldehyde synthesis, up-regulation of chanoclavine-I aldehyde anabolism, up-regulation of chanoclavine-I aldehyde biosynthesis, up-regulation of chanoclavine-I aldehyde biosynthetic process, up-regulation of chanoclavine-I aldehyde formation, up-regulation of chanoclavine-I aldehyde synthesis, upregulation of chanoclavine-I aldehyde anabolism, upregulation of chanoclavine-I aldehyde biosynthesis, upregulation of chanoclavine-I aldehyde biosynthetic process, upregulation of chanoclavine-I aldehyde formation, upregulation of chanoclavine-I aldehyde synthesis, activation of chanoclavine-I aldehyde biosynthetic process Relationships: is a type of regulation of chanoclavine-I aldehyde biosynthetic process [GO:1900646]; is a type of positive regulation of ergot alkaloid biosynthetic process [GO:1900824]; positively regulates chanoclavine-I aldehyde biosynthetic process [GO:1900569]